{
  "term_label": "Unknown cellular component",
  "gene_name": "Protein NOXP20",
  "gene_symbol": "FAM114A1",
  "term_id": "UNKNOWN:0003",
  "gene": "UniProtKB:Q8IWE2"
}